{
  "gene_symbol": "CMAHP",
  "gene": "UniProtKB:Q9Y471",
  "gene_name": "Inactive cytidine monophosphate-N-acetylneuraminic acid hydroxylase",
  "term_id": "GO:0030338",
  "term_label": "CMP-N-acetylneuraminate monooxygenase activity"
}